{
  "term_label": "GTPase activator activity",
  "gene": "UniProtKB:Q8IYB5",
  "gene_name": "Stromal membrane-associated protein 1",
  "term_id": "GO:0005096",
  "gene_symbol": "SMAP1"
}